regulation of DNA recombination at centromere [GO:0061806] (biological process) Subtypes: positive regulation of DNA recombination at centromere [GO:0061807], negative regulation of DNA recombination at centromere [GO:0061808] Definition: Any process that modulates the frequency, rate or extent of DNA recombination within centromeric DNA. Relationships: is a type of GO:0000018 References: PMID:27697832 Sources: GOC:dph, GOC:mah Also known as: regulation of centromeric recombination